regulation of nigerotriose transport [GO:1900357] (biological process) Definition: Any process that modulates the frequency, rate or extent of nigerotriose transport. Subtypes: negative regulation of nigerotriose transport [GO:1900358], positive regulation of nigerotriose transport [GO:1900359] Relationships: is a type of regulation of transport [GO:0051049]; regulates nigerotriose transport [GO:2001091] Sources: GOC:TermGenie, GOC:mengo_curators